6-sulfoquinovose(1-) catabolic process to 3-sulfopropanediol(1-) [GO:0061721] (biological process) References: PMID:14602517, PMID:24463506 Sources: GOC:dph Definition: The chemical reactions and pathways resulting in the breakdown of 6-sulfoquinovose(1-) resulting in the formation of glycerone phosphate (DHAP) and 3-sulfopropanediol(1-). Relationships: is_a GO:0019694; is a type of glycol metabolic process [GO:0042844]; is a type of 6-sulfoquinovose(1-) catabolic process [GO:1902777]; has part 3-sulfolactaldehyde reductase activity [GO:0061596]; has part 6-sulfoquinovose(1-) catabolic process to glycerone phosphate and 3-sulfolactaldehyde [GO:0061720]